ABC-type ferric-enterobactin transporter activity [GO:0015624] (molecular function) Definition: Enables the transfer of a solute or solutes from one side of a membrane to the other according to the reaction: ATP + H2O + ferric-enterobactin(out) = ADP + phosphate + ferric-enterobactin(in). Sources: RHEA:58492 Also known as: ferric-enterobactin porter activity, ATP-dependent ferric-enterobactin transmembrane transporter activity, ferric-enterobactin ABC transporter, ATPase-coupled ferric-enterobactin transmembrane transporter activity, ferric-enterobactin-transporting ATPase activity Relationships: is a type of iron chelate transmembrane transporter activity [GO:0015603]; is a type of ABC-type transporter activity [GO:0140359]